positive regulation of growth rate [GO:0040010] (biological process) Also known as: up regulation of growth rate, up-regulation of growth rate, upregulation of growth rate, activation of growth rate, stimulation of growth rate Relationships: is_a regulation of growth rate [GO:0040009]; is a type of GO:0045927 Sources: GOC:mah Definition: Any process that increases the rate of growth of all or part of an organism. Note: Note that this term and its definition depart from the usual conventions for GO 'regulation' process terms; regulation of rate is not usually distinguished from regulation of extent or frequency, but it makes sense to do so for growth regulation.